{
  "gene": "UniProtKB:Q9NPB9",
  "gene_symbol": "ACKR4",
  "gene_name": "Atypical chemokine receptor 4",
  "term_id": "GO:0006955",
  "term_label": "immune response"
}